{
  "gene_symbol": "AIM2",
  "term_label": "cellular response to interferon-beta",
  "gene_name": "Interferon-inducible protein AIM2",
  "gene": "UniProtKB:O14862",
  "term_id": "GO:0035458"
}